{
  "gene_symbol": "SLFN12L",
  "gene_name": "Schlafen family member 12-like",
  "gene": "UniProtKB:Q6IEE8",
  "term_id": "UNKNOWN:0002",
  "term_label": "Unknown biological process"
}